{
  "gene": "UniProtKB:Q8N4B1",
  "gene_symbol": "PHETA1",
  "term_label": "endosome organization",
  "term_id": "GO:0007032",
  "gene_name": "Sesquipedalian-1"
}